{
  "gene_symbol": "LMO7DN",
  "gene": "UniProtKB:F2Z398",
  "gene_name": "LMO7 downstream neighbor protein",
  "term_label": "Unknown molecular function",
  "term_id": "UNKNOWN:0001"
}